{
  "term_label": "crossover junction DNA endonuclease activity",
  "term_id": "GO:0008821",
  "gene": "UniProtKB:O43502",
  "gene_name": "DNA repair protein RAD51 homolog 3",
  "gene_symbol": "RAD51C"
}